{
  "gene_name": "UDP-glucuronosyltransferase 1A3",
  "gene_symbol": "UGT1A3",
  "gene": "UniProtKB:P35503",
  "term_label": "flavone metabolic process",
  "term_id": "GO:0051552"
}